{
  "term_id": "GO:0001654",
  "gene_symbol": "MEIS3P2",
  "term_label": "eye development",
  "gene": "UniProtKB:A8K0S8",
  "gene_name": "Putative homeobox protein Meis3-like 2"
}